{
  "gene_symbol": "NHERF4",
  "term_label": "protein localization to plasma membrane",
  "gene": "UniProtKB:Q86UT5",
  "term_id": "GO:0072659",
  "gene_name": "Na(+)_H(+) exchange regulatory cofactor NHE-RF4"
}